{
  "term_id": "GO:0012505",
  "gene_symbol": "RAB18",
  "term_label": "endomembrane system",
  "gene": "UniProtKB:Q9NP72",
  "gene_name": "Ras-related protein Rab-18"
}